{
  "gene_symbol": "SLC12A8",
  "term_id": "GO:0055075",
  "gene": "UniProtKB:A0AV02",
  "term_label": "potassium ion homeostasis",
  "gene_name": "Solute carrier family 12 member 8"
}